{
  "gene_name": "Putative uncharacterized protein DHRS4-AS1",
  "term_id": "UNKNOWN:0002",
  "term_label": "Unknown biological process",
  "gene_symbol": "DHRS4-AS1",
  "gene": "UniProtKB:Q9P1J3"
}